{
  "gene_name": "E3 ubiquitin-protein ligase HERC2",
  "gene": "UniProtKB:O95714",
  "term_label": "protein ubiquitination",
  "term_id": "GO:0016567",
  "gene_symbol": "HERC2"
}